{
  "term_id": "GO:0006890",
  "gene": "UniProtKB:Q8TD16",
  "gene_name": "Protein bicaudal D homolog 2",
  "term_label": "retrograde vesicle-mediated transport, Golgi to endoplasmic reticulum",
  "gene_symbol": "BICD2"
}